{
  "term_label": "mRNA splicing, via spliceosome",
  "gene": "UniProtKB:Q13838",
  "gene_name": "Spliceosome RNA helicase DDX39B",
  "gene_symbol": "DDX39B",
  "term_id": "GO:0000398"
}